{
  "term_id": "GO:0048019",
  "gene_name": "Humanin-like 1",
  "gene": "UniProtKB:P0CJ68",
  "gene_symbol": "MTRNR2L1",
  "term_label": "receptor antagonist activity"
}